negative regulation of motor neuron apoptotic process [GO:2000672] (biological process) Definition: Any process that stops, prevents or reduces the frequency, rate or extent of motor neuron apoptotic process. Sources: GOC:mtg_apoptosis, GOC:obol Also known as: negative regulation of motoneuron apoptosis, negative regulation of motor neuron apoptosis Relationships: is a type of negative regulation of neuron apoptotic process [GO:0043524]; is a type of GO:2000671; negatively regulates GO:0097049